{
  "gene_name": "C-X-C motif chemokine 17",
  "term_id": "GO:0048246",
  "gene": "UniProtKB:Q6UXB2",
  "gene_symbol": "CXCL17",
  "term_label": "macrophage chemotaxis"
}